{
  "term_id": "GO:0004132",
  "gene_name": "Cytidine and dCMP deaminase domain-containing protein 1",
  "gene_symbol": "CDADC1",
  "term_label": "dCMP deaminase activity",
  "gene": "UniProtKB:Q9BWV3"
}